{
  "gene_name": "YY1-associated factor 2",
  "gene_symbol": "YAF2",
  "term_id": "GO:0006355",
  "term_label": "regulation of DNA-templated transcription",
  "gene": "UniProtKB:Q8IY57"
}